{
  "term_label": "photoreceptor outer segment",
  "gene_name": "Opsin-5",
  "term_id": "GO:0001750",
  "gene": "UniProtKB:Q6U736",
  "gene_symbol": "OPN5"
}